{
  "gene_symbol": "ABI1",
  "term_id": "GO:0035591",
  "term_label": "signaling adaptor activity",
  "gene_name": "Abl interactor 1",
  "gene": "UniProtKB:Q8IZP0"
}